{
  "term_label": "plasma membrane",
  "gene_name": "Ammonium transporter Rh type C",
  "term_id": "GO:0005886",
  "gene_symbol": "RHCG",
  "gene": "UniProtKB:Q9UBD6"
}